{
  "gene_symbol": "STIM1",
  "term_label": "calcium channel regulator activity",
  "gene": "UniProtKB:Q13586",
  "gene_name": "Stromal interaction molecule 1",
  "term_id": "GO:0005246"
}